{
  "term_id": "GO:0043328",
  "term_label": "protein transport to vacuole involved in ubiquitin-dependent protein catabolic process via the multivesicular body sorting pathway",
  "gene": "UniProtKB:Q86VN1",
  "gene_symbol": "VPS36",
  "gene_name": "Vacuolar protein-sorting-associated protein 36"
}